{
  "gene_name": "Microtubule-associated serine_threonine-protein kinase 2",
  "term_label": "microtubule binding",
  "term_id": "GO:0008017",
  "gene": "UniProtKB:Q6P0Q8",
  "gene_symbol": "MAST2"
}